{
  "gene_name": "Protein PML",
  "gene": "UniProtKB:P29590",
  "term_label": "ubiquitin-like protein ligase activity",
  "gene_symbol": "PML",
  "term_id": "GO:0061659"
}